{
  "gene": "UniProtKB:P42785",
  "gene_name": "Lysosomal Pro-X carboxypeptidase",
  "term_label": "Unknown cellular component",
  "gene_symbol": "PRCP",
  "term_id": "UNKNOWN:0003"
}